{
  "gene": "UniProtKB:A6NG13",
  "gene_name": "Alpha-1,3-mannosyl-glycoprotein 4-beta-N-acetylglucosaminyltransferase-like protein MGAT4D",
  "term_label": "endoplasmic reticulum-Golgi intermediate compartment",
  "term_id": "GO:0005793",
  "gene_symbol": "MGAT4D"
}